{
  "gene_name": "Trefoil factor 3",
  "gene_symbol": "TFF3",
  "term_label": "maintenance of gastrointestinal epithelium",
  "term_id": "GO:0030277",
  "gene": "UniProtKB:Q07654"
}